cellular response to carbendazim [GO:0072762] (biological process) Relationships: is_a response to carbendazim [GO:1901597] Definition: Any process that results in a change in state or activity of a cell (in terms of movement, secretion, enzyme production, gene expression, etc.) as a result of a carbendazim stimulus. Sources: GOC:mah